{
  "gene_name": "Angiopoietin-1 receptor",
  "gene_symbol": "TEK",
  "term_label": "angiogenesis",
  "gene": "UniProtKB:Q02763",
  "term_id": "GO:0001525"
}